{
  "term_label": "actin filament",
  "gene": "UniProtKB:Q13459",
  "gene_name": "Unconventional myosin-IXb",
  "gene_symbol": "MYO9B",
  "term_id": "GO:0005884"
}